{
  "term_id": "GO:0003712",
  "gene_symbol": "RAI1",
  "gene": "UniProtKB:Q7Z5J4",
  "term_label": "transcription coregulator activity",
  "gene_name": "Retinoic acid-induced protein 1"
}